{
  "term_id": "GO:0005829",
  "term_label": "cytosol",
  "gene_symbol": "PGD",
  "gene": "UniProtKB:P52209",
  "gene_name": "6-phosphogluconate dehydrogenase, decarboxylating"
}